{
  "gene": "UniProtKB:Q15306",
  "gene_name": "Interferon regulatory factor 4",
  "term_id": "GO:0000978",
  "gene_symbol": "IRF4",
  "term_label": "RNA polymerase II cis-regulatory region sequence-specific DNA binding"
}